{
  "term_label": "extracellular region",
  "gene_name": "Progranulin",
  "term_id": "GO:0005576",
  "gene": "UniProtKB:P28799",
  "gene_symbol": "GRN"
}